{
  "term_id": "GO:0004082",
  "gene": "UniProtKB:P07738",
  "term_label": "bisphosphoglycerate mutase activity",
  "gene_symbol": "BPGM",
  "gene_name": "Bisphosphoglycerate mutase"
}